{
  "term_id": "GO:0000118",
  "gene": "UniProtKB:Q9UKL0",
  "gene_name": "REST corepressor 1",
  "term_label": "histone deacetylase complex",
  "gene_symbol": "RCOR1"
}